{
  "gene_symbol": "AKAP4",
  "gene_name": "A-kinase anchor protein 4",
  "gene": "UniProtKB:Q5JQC9",
  "term_label": "sperm principal piece",
  "term_id": "GO:0097228"
}